{
  "term_label": "actin filament organization",
  "gene_symbol": "TRPV3",
  "gene_name": "Transient receptor potential cation channel subfamily V member 3",
  "term_id": "GO:0007015",
  "gene": "UniProtKB:Q8NET8"
}